somatic diversification of immune receptors via gene conversion [GO:0002565] (biological process) Sources: GOC:add, ISBN:0781735149 Relationships: is a type of somatic diversification of immune receptors [GO:0002200]; is a type of GO:0016444 Definition: The process in which immune receptor genes are diversified through gene conversion. Subtypes: GO:0002206